apical plasma membrane [GO:0016324] (cellular component) Definition: The region of the plasma membrane located at the apical end of the cell. Sources: GOC:curators Relationships: is_a plasma membrane region [GO:0098590]; is part of GO:0045177